TTP biosynthetic process [GO:0006234] (biological process) Sources: ISBN:0198506732 Also known as: TTP anabolism, TTP biosynthesis, TTP formation, TTP synthesis Relationships: is a type of pyrimidine ribonucleoside triphosphate biosynthetic process [GO:0009209]; is a type of pyrimidine ribonucleotide biosynthetic process [GO:0009220]; is_a TTP metabolic process [GO:0046046] Definition: The chemical reactions and pathways resulting in the formation of TTP, ribosylthymine triphosphate.